{
  "gene": "UniProtKB:Q9UJM3",
  "gene_symbol": "ERRFI1",
  "term_label": "Unknown cellular component",
  "gene_name": "ERBB receptor feedback inhibitor 1",
  "term_id": "UNKNOWN:0003"
}